{
  "gene": "UniProtKB:Q6UWF3",
  "gene_symbol": "SCIMP",
  "gene_name": "SLP adapter and CSK-interacting membrane protein",
  "term_id": "GO:0001772",
  "term_label": "immunological synapse"
}